linalool 8-monooxygenase activity [GO:0050056] (molecular function) Definition: Catalysis of the reaction: linalool + 2 O2 + 2 reduced [NADPH--hemoprotein reductase] = (6E)-8-oxolinalool + 2 H+ + 3 H2O + 2 oxidized [NADPH--hemoprotein reductase]. Sources: RHEA:32635 Also known as: linalool,[reduced NADPH--hemoprotein reductase]:oxygen oxidoreductase (8-hydroxylating) activity Relationships: is a type of oxidoreductase activity, acting on paired donors, with incorporation or reduction of molecular oxygen, reduced flavin or flavoprotein as one donor, and incorporation of one atom of oxygen [GO:0016712]